{
  "term_id": "UNKNOWN:0001",
  "gene_name": "Putative uncharacterized protein encoded by ERC2-IT1",
  "gene_symbol": "ERC2-IT1",
  "term_label": "Unknown molecular function",
  "gene": "UniProtKB:O76042"
}